{
  "gene_name": "ERI1 exoribonuclease 2",
  "gene": "UniProtKB:A8K979",
  "term_id": "GO:0060906",
  "term_label": "negative regulation of regulatory ncRNA-mediated heterochromatin formation",
  "gene_symbol": "ERI2"
}